{
  "gene_symbol": "KCNA3",
  "gene": "UniProtKB:P22001",
  "gene_name": "Potassium voltage-gated channel subfamily A member 3",
  "term_id": "GO:0008076",
  "term_label": "voltage-gated potassium channel complex"
}